{
  "gene_name": "TBC1 domain family member 22B",
  "term_id": "UNKNOWN:0002",
  "term_label": "Unknown biological process",
  "gene": "UniProtKB:Q9NU19",
  "gene_symbol": "TBC1D22B"
}